{
  "gene": "UniProtKB:Q2VPJ9",
  "term_label": "Unknown cellular component",
  "gene_name": "Leucine-rich repeat-containing protein 75B",
  "term_id": "UNKNOWN:0003",
  "gene_symbol": "LRRC75B"
}